{
  "term_label": "excitatory extracellular ligand-gated monoatomic ion channel activity",
  "gene_name": "5-hydroxytryptamine receptor 3E",
  "gene": "UniProtKB:A5X5Y0",
  "gene_symbol": "HTR3E",
  "term_id": "GO:0005231"
}